antipodal cell nucleus [GO:0043079] (cellular component) Sources: CL:0000537, GOC:jl Definition: The nucleus of an antipodal cell, one of three cells of the embryo sac in angiosperms, found at the chalazal end of the embryo away from the point of entry of the pollen tube, and its descendents. Relationships: is a type of GO:0043076